{
  "gene_symbol": "PSG1",
  "term_label": "Unknown cellular component",
  "gene": "UniProtKB:P11464",
  "term_id": "UNKNOWN:0003",
  "gene_name": "Pregnancy-specific beta-1-glycoprotein 1"
}